pyrimidine nucleotide transport [GO:0006864] (biological process) Definition: The directed movement of a pyrimidine nucleotide, any compound consisting of a pyrimidine nucleoside esterified with (ortho)phosphate, into, out of or within a cell. Sources: GOC:ai Subtypes: pyrimidine nucleotide import into mitochondrion [GO:1990519] Relationships: is a type of nucleotide transport [GO:0006862]